D-benzoylarginine-4-nitroanilide amidase activity [GO:0047415] (molecular function) Relationships: is a type of GO:0016811 Also known as: D-BAPA-ase activity, N-benzoyl-D-arginine-4-nitroanilide amidohydrolase activity, benzoyl-D-arginine arylamidase activity Definition: Catalysis of the reaction: N(2)-benzoyl-D-arginine-4-nitroanilide + H2O = 4-nitroaniline + N(2)-benzoyl-D-arginine + H+. Sources: EC:3.5.1.72, RHEA:14421